heme binding [GO:0020037] (molecular function) Definition: Binding to a heme, a compound composed of iron complexed in a porphyrin (tetrapyrrole) ring. Relationships: is a type of tetrapyrrole binding [GO:0046906] Sources: GOC:ai Also known as: haem binding